{
  "gene_symbol": "TRBV29-1",
  "gene_name": "T cell receptor beta variable 29-1",
  "term_label": "plasma membrane",
  "gene": "UniProtKB:A0A5B7",
  "term_id": "GO:0005886"
}